Mo(VI)-molybdopterin cytosine dinucleotide biosynthetic process [GO:1902760] (biological process) References: PMID:23201473 Sources: GOC:TermGenie, GOC:dph, GO_REF:0000068 Also known as: Mo(VI)-molybdopterin cytosine dinucleotide anabolism, Mo(VI)-molybdopterin cytosine dinucleotide biosynthesis, Mo(VI)-molybdopterin cytosine dinucleotide formation, Mo(VI)-molybdopterin cytosine dinucleotide synthesis, Mo-molybdopterin-cytosine-dinucleotide cofactor biosynthetic process Definition: The chemical reactions and pathways resulting in the formation of Mo(VI)-molybdopterin cytosine dinucleotide. Relationships: is_a Mo-molybdopterin cofactor biosynthetic process [GO:0006777]; has part molybdenum cofactor cytidylyltransferase activity [GO:0061602]